{
  "gene_name": "Cytohesin-2",
  "term_id": "GO:0016192",
  "gene_symbol": "CYTH2",
  "term_label": "vesicle-mediated transport",
  "gene": "UniProtKB:Q99418"
}